{
  "term_id": "GO:0019911",
  "gene_symbol": "PLP1",
  "gene_name": "Myelin proteolipid protein",
  "gene": "UniProtKB:P60201",
  "term_label": "structural constituent of myelin sheath"
}